{
  "gene_symbol": "UTP14A",
  "term_id": "GO:0005730",
  "term_label": "nucleolus",
  "gene_name": "U3 small nucleolar RNA-associated protein 14 homolog A",
  "gene": "UniProtKB:Q9BVJ6"
}